{
  "gene_symbol": "GPR32P1",
  "gene_name": "Putative G-protein coupled receptor GPR32P1",
  "term_id": "GO:0007204",
  "gene": "UniProtKB:Q8NGA4",
  "term_label": "positive regulation of cytosolic calcium ion concentration"
}